RNA cap trimethylguanosine synthase activity [GO:0071164] (molecular function) Definition: Catalysis of two successive methyl transfer reactions from AdoMet to the N-2 atom of guanosine, thereby converting 7-methylguanosine in an RNA cap to 2,2,7 trimethylguanosine. References: PMID:11983179, PMID:18775984 Also known as: RNA trimethylguanosine synthase activity, cap hypermethylase activity, small nuclear RNA methyltransferase activity, snRNA methyltransferase activity Note: A 2,2,7-trimethylguanosine (TMG) cap is found on many RNA polymerase II transcribed small noncoding RNAs including small nuclear RNA (snRNA), small nucleolar RNA (snoRNA) and telomerase RNA. It is also found on nematode mRNAs that undergo trans-splicing of a 5'-capped leader sequence. Relationships: is a type of RNA methyltransferase activity [GO:0008173]; is a type of S-adenosylmethionine-dependent methyltransferase activity [GO:0008757]; is part of 7-methylguanosine cap hypermethylation [GO:0036261]